{
  "gene": "UniProtKB:P22466",
  "term_id": "GO:0007218",
  "gene_name": "Galanin peptides",
  "gene_symbol": "GAL",
  "term_label": "neuropeptide signaling pathway"
}